{
  "gene": "UniProtKB:A0A0B4J244",
  "gene_name": "T cell receptor alpha variable 3",
  "gene_symbol": "TRAV3",
  "term_id": "GO:0002250",
  "term_label": "adaptive immune response"
}